{
  "gene_name": "Transportin-1",
  "gene_symbol": "TNPO1",
  "term_label": "nucleus",
  "term_id": "GO:0005634",
  "gene": "UniProtKB:Q92973"
}